{
  "gene_name": "Ras-related protein Rap-1b",
  "gene_symbol": "RAP1B",
  "term_id": "GO:0071320",
  "term_label": "cellular response to cAMP",
  "gene": "UniProtKB:P61224"
}